positive regulation of morphogenesis of an epithelium [GO:1905332] (biological process) Subtypes: prostate induction [GO:0060514], GO:0060787, GO:0061047, renal vesicle induction [GO:0072034], GO:0072108, GO:0090190, positive regulation of heart looping [GO:1901209], positive regulation of convergent extension involved in axis elongation [GO:1901234], positive regulation of epiboly involved in gastrulation with mouth forming second [GO:1904088], GO:1904105, positive regulation of otic vesicle morphogenesis [GO:1904120], GO:1905278, GO:1905555, GO:1905956 References: PMID:25745997 Sources: GOC:TermGenie, GOC:bhm, GO_REF:0000058 Relationships: is a type of positive regulation of developmental process [GO:0051094]; is_a regulation of morphogenesis of an epithelium [GO:1905330]; positively regulates GO:0002009 Also known as: positive regulation of epithelium morphogenesis, up regulation of epithelium morphogenesis, up regulation of morphogenesis of an epithelium, up-regulation of epithelium morphogenesis, up-regulation of morphogenesis of an epithelium, upregulation of epithelium morphogenesis, upregulation of morphogenesis of an epithelium, activation of epithelium morphogenesis, activation of morphogenesis of an epithelium Definition: Any process that activates or increases the frequency, rate or extent of morphogenesis of an epithelium. Note: An example of this is MMRN2 in human (Q9H8L6) in PMID:25745997 (inferred from direct assay).